{
  "gene_name": "Putative uncharacterized protein encoded by RHPN1-AS1",
  "gene": "UniProtKB:Q9BWJ2",
  "gene_symbol": "RHPN1-AS1",
  "term_id": "UNKNOWN:0001",
  "term_label": "Unknown molecular function"
}